{
  "gene_name": "Leukocyte cell-derived chemotaxin 1",
  "gene": "UniProtKB:O75829",
  "gene_symbol": "CNMD",
  "term_id": "UNKNOWN:0001",
  "term_label": "Unknown molecular function"
}